attachment of spindle microtubules to kinetochore [GO:0008608] (BP) Note: This class covers all attachments of spindle microtubules to the kinetochore, including the many incorrect attachments which initially form and are later corrected to stable attachments with the correct orientation for segregation to proceed (sister chromatid biorientation). Definition: The process in which spindle microtubules become physically associated with the proteins making up the kinetochore complex. Regulation: negatively regulated by negative regulation of attachment of spindle microtubules to kinetochore [GO:0051986]; positively regulated by GO:0051987; RO_0002211 by regulation of attachment of spindle microtubules to kinetochore [GO:0051988] Also known as: kinetochore microtubule interaction, kinetochore-microtubule interaction, microtubule and chromosome interaction, spindle-chromosome interaction, attachment of spindle microtubules to chromosome, kinetochore-microtubule attachment, microtubule anchoring at kinetochore, spindle chromosome attachment, spindle kinetochore attachment, microtubule capture, amphotelic attachment, bipolar attachment, microtubule and kinetochore interaction References: PMID:10322137 Sources: GOC:vw Subtypes: sister chromatid biorientation [GO:0031134], attachment of mitotic spindle microtubules to kinetochore [GO:0051315], attachment of meiotic spindle microtubules to kinetochore [GO:0051316] Relationships: is a type of cell cycle process [GO:0022402]; is part of metaphase chromosome alignment [GO:0051310]; has part microtubule binding [GO:0008017]